{
  "gene": "UniProtKB:Q96F83",
  "term_id": "GO:0030276",
  "gene_symbol": "CLBA1",
  "gene_name": "Uncharacterized protein CLBA1",
  "term_label": "clathrin binding"
}